{
  "gene": "UniProtKB:P0CG24",
  "gene_name": "Zinc finger protein 883",
  "term_id": "UNKNOWN:0003",
  "gene_symbol": "ZNF883",
  "term_label": "Unknown cellular component"
}